{
  "gene_symbol": "YY2",
  "term_label": "regulation of transcription by RNA polymerase II",
  "gene": "UniProtKB:O15391",
  "term_id": "GO:0006357",
  "gene_name": "Transcription factor YY2"
}